multi-eIF complex [GO:0043614] (cellular component) Also known as: multifactor translation initiation factor (eIF) complex Relationships: is a type of ribonucleoprotein complex [GO:1990904]; is part of cytoplasm [GO:0005737] Sources: GOC:krc Definition: A multifactor complex composed of multiple translation initiation factors and the initiatior tRNAiMet, which is ready to bind to the small (40S) ribosome to form the 43S preinitiation complex. In S. cerevisiae, this complex is composed of eIF1, eIF2, eIF3, and eIF5.